{
  "term_label": "cell division",
  "gene_name": "Anaphase-promoting complex subunit 7",
  "term_id": "GO:0051301",
  "gene": "UniProtKB:Q9UJX3",
  "gene_symbol": "ANAPC7"
}